{
  "gene_name": "Putative uncharacterized protein encoded by AGPAT4-IT1",
  "term_label": "Unknown molecular function",
  "term_id": "UNKNOWN:0001",
  "gene": "UniProtKB:Q9H0P7",
  "gene_symbol": "AGPAT4-IT1"
}